{
  "term_label": "positive regulation of cell population proliferation",
  "term_id": "GO:0008284",
  "gene": "UniProtKB:P48357",
  "gene_name": "Leptin receptor",
  "gene_symbol": "LEPR"
}